{
  "gene_symbol": "TAL1",
  "gene_name": "T-cell acute lymphocytic leukemia protein 1",
  "term_label": "regulation of transcription by RNA polymerase II",
  "term_id": "GO:0006357",
  "gene": "UniProtKB:P17542"
}